{
  "gene_symbol": "SELENOW",
  "gene": "UniProtKB:P63302",
  "term_id": "UNKNOWN:0001",
  "gene_name": "Selenoprotein W",
  "term_label": "Unknown molecular function"
}